{
  "gene_name": "T-box transcription factor TBX3",
  "gene": "UniProtKB:O15119",
  "term_id": "GO:0005634",
  "term_label": "nucleus",
  "gene_symbol": "TBX3"
}